{
  "term_label": "Unknown molecular function",
  "gene_name": "Putative protein FAM90A2P",
  "gene": "UniProtKB:Q658T7",
  "term_id": "UNKNOWN:0001",
  "gene_symbol": "FAM90A2P"
}